{
  "term_label": "axon",
  "gene_symbol": "CALCR",
  "gene": "UniProtKB:P30988",
  "term_id": "GO:0030424",
  "gene_name": "Calcitonin receptor"
}